maleimide hydrolase activity [GO:0050539] (molecular function) Also known as: imidase activity, cyclic imide hydrolase activity, cyclic-imide amidohydrolase (decyclicizing), cyclic-imide amidohydrolase (decyclizing) Relationships: is_a hydrolase activity, acting on carbon-nitrogen (but not peptide) bonds, in cyclic amides [GO:0016812] Sources: EC:3.5.2.16, RHEA:24476 Definition: Catalysis of the reaction: H2O + maleimide = H+ + maleamate.